{
  "gene_name": "ETS-related transcription factor Elf-5",
  "term_label": "DNA-binding transcription factor activity, RNA polymerase II-specific",
  "gene": "UniProtKB:Q9UKW6",
  "term_id": "GO:0000981",
  "gene_symbol": "ELF5"
}